positive regulation of stem cell proliferation [GO:2000648] (biological process) Relationships: is a type of positive regulation of cell population proliferation [GO:0008284]; is a type of regulation of stem cell proliferation [GO:0072091]; positively regulates stem cell proliferation [GO:0072089] Definition: Any process that activates or increases the frequency, rate or extent of stem cell proliferation. Sources: GOC:dph Subtypes: positive regulation of hematopoietic stem cell proliferation [GO:1902035], positive regulation of mesenchymal stem cell proliferation [GO:1902462]